{
  "gene_name": "Probable crossover junction endonuclease EME2",
  "gene_symbol": "EME2",
  "term_id": "GO:0006302",
  "gene": "UniProtKB:A4GXA9",
  "term_label": "double-strand break repair"
}